positive regulation of relaxation of muscle [GO:1901079] (BP) Also known as: up regulation of relaxation of muscle, up-regulation of relaxation of muscle, upregulation of relaxation of muscle, activation of relaxation of muscle Definition: Any process that activates or increases the frequency, rate or extent of relaxation of muscle. Relationships: is_a positive regulation of multicellular organismal process [GO:0051240]; is a type of GO:1901077; positively regulates GO:0090075 Sources: GOC:TermGenie Subtypes: positive regulation of relaxation of smooth muscle [GO:1901082], GO:1901899